{
  "term_label": "6-phosphogluconolactonase activity",
  "gene": "UniProtKB:O95336",
  "term_id": "GO:0017057",
  "gene_name": "6-phosphogluconolactonase",
  "gene_symbol": "PGLS"
}